cell wall organization or biogenesis [GO:0071554] (BP) Also known as: cell wall organisation or biogenesis, cell wall organization or biogenesis at cellular level, cellular cell wall organisation or biogenesis, cellular cell wall organization or biogenesis Relationships: is a type of GO:0009987 Sources: GOC:mah Subtypes: cell wall biogenesis [GO:0042546], GO:0071555, plant-type cell wall organization or biogenesis [GO:0071669], fungal-type cell wall organization or biogenesis [GO:0071852] Definition: A process that results in the biosynthesis of constituent macromolecules, assembly, arrangement of constituent parts, or disassembly of a cell wall. Regulation: regulated by regulation of cell wall organization or biogenesis [GO:1903338]; RO_0002212 by negative regulation of cell wall organization or biogenesis [GO:1903339]; positively regulated by positive regulation of cell wall organization or biogenesis [GO:1903340]